{
  "term_id": "GO:0031209",
  "gene_symbol": "BRK1",
  "gene_name": "Protein BRICK1",
  "gene": "UniProtKB:Q8WUW1",
  "term_label": "SCAR complex"
}